{
  "gene_symbol": "OBSCN",
  "term_id": "UNKNOWN:0002",
  "gene": "UniProtKB:Q5VST9",
  "gene_name": "Obscurin",
  "term_label": "Unknown biological process"
}